{
  "gene_symbol": "KCNN2",
  "gene_name": "Small conductance calcium-activated potassium channel protein 2",
  "gene": "UniProtKB:Q9H2S1",
  "term_label": "small conductance calcium-activated potassium channel activity",
  "term_id": "GO:0016286"
}